{
  "gene_symbol": "PTPRS",
  "term_label": "Unknown cellular component",
  "gene_name": "Receptor-type tyrosine-protein phosphatase S",
  "term_id": "UNKNOWN:0003",
  "gene": "UniProtKB:Q13332"
}